{
  "gene": "UniProtKB:Q9NS00",
  "term_id": "UNKNOWN:0002",
  "gene_name": "Glycoprotein-N-acetylgalactosamine 3-beta-galactosyltransferase 1",
  "gene_symbol": "C1GALT1",
  "term_label": "Unknown biological process"
}